cutin biosynthetic process [GO:0010143] (biological process) Definition: The chemical reactions and pathways resulting in the formation of cutin, a waxy substance, which combined with cellulose forms a substance nearly impervious to water and constituting the cuticle in plants. Sources: ISBN:0028623819 Also known as: cutin anabolism, cutin biosynthesis, cutin formation, cutin synthesis Relationships: is a type of macromolecule biosynthetic process [GO:0009059]; is part of cutin-based cuticle development [GO:0160062] Regulation: regulated by regulation of cutin biosynthetic process [GO:1901957]; negatively regulated by negative regulation of cutin biosynthetic process [GO:1901958]; positively regulated by positive regulation of cutin biosynthetic process [GO:1901959]